{
  "term_label": "positive regulation of nuclear-transcribed mRNA poly(A) tail shortening",
  "term_id": "GO:0060213",
  "gene": "UniProtKB:Q9HCJ0",
  "gene_name": "Trinucleotide repeat-containing gene 6C protein",
  "gene_symbol": "TNRC6C"
}